GDP-mannose metabolic process [GO:0019673] (biological process) Definition: The chemical reactions and pathways involving GDP-mannose, a substance composed of mannose in glycosidic linkage with guanosine diphosphate. Sources: GOC:ai Also known as: GDP-mannose metabolism Relationships: is a type of nucleotide-sugar metabolic process [GO:0009225] Subtypes: GDP-mannose biosynthetic process [GO:0009298], GO:0042351